glucocorticoid biosynthetic process [GO:0006704] (biological process) Definition: The chemical reactions and pathways resulting in the formation of glucocorticoids, hormonal C21 corticosteroids synthesized from cholesterol. Sources: ISBN:0198506732 Also known as: glucocorticoid anabolism, glucocorticoid biosynthesis, glucocorticoid formation, glucocorticoid synthesis Relationships: is a type of glucocorticoid metabolic process [GO:0008211]; is a type of steroid hormone biosynthetic process [GO:0120178] Subtypes: cortisol biosynthetic process [GO:0034651] Regulation: regulated by regulation of glucocorticoid biosynthetic process [GO:0031946]; negatively regulated by GO:0031947; positively regulated by positive regulation of glucocorticoid biosynthetic process [GO:0031948]